{
  "gene": "UniProtKB:P29965",
  "term_id": "GO:0005615",
  "term_label": "extracellular space",
  "gene_name": "CD40 ligand",
  "gene_symbol": "CD40LG"
}